late endosome to lysosome transport via multivesicular body sorting pathway [GO:0061764] (BP) Sources: GOC:dph Definition: The directed movement of substances from late endosomes to lysosomes by a pathway in which molecules are sorted into multivesicular bodies, which then fuse with the lysosome. Relationships: is a type of endosome to lysosome transport via multivesicular body sorting pathway [GO:0032510]; is a type of GO:0045324; is a type of late endosome to lysosome transport [GO:1902774]